{
  "gene": "UniProtKB:Q96DA0",
  "term_label": "Unknown molecular function",
  "term_id": "UNKNOWN:0001",
  "gene_name": "Zymogen granule protein 16 homolog B",
  "gene_symbol": "ZG16B"
}